mesonephric nephron tubule development [GO:0061242] (biological process) Sources: GOC:mtg_kidney_jan10 Relationships: is a type of GO:0061241; is a type of nephron tubule development [GO:0072080]; is a type of mesonephric tubule development [GO:0072164] Subtypes: mesonephric connecting tubule development [GO:0061272], mesonephric distal tubule development [GO:0061274], mesonephric proximal tubule development [GO:0061275] Definition: The progression of a mesonephric nephron tubule over time, from its initial formation to the mature structure. A mesonephric nephron tubule is an epithelial tube that is part of the mesonephric nephron, the functional part of the mesonephros.